{
  "gene_symbol": "DAG1",
  "term_id": "GO:0042383",
  "gene": "UniProtKB:Q14118",
  "term_label": "sarcolemma",
  "gene_name": "Dystroglycan 1"
}